{
  "term_id": "GO:0002486",
  "gene_symbol": "RAET1L",
  "gene_name": "UL16-binding protein 6",
  "term_label": "antigen processing and presentation of endogenous peptide antigen via MHC class I via ER pathway, TAP-independent",
  "gene": "UniProtKB:Q5VY80"
}